{
  "term_id": "GO:0003690",
  "gene": "UniProtKB:Q06609",
  "gene_name": "DNA repair protein RAD51 homolog 1",
  "gene_symbol": "RAD51",
  "term_label": "double-stranded DNA binding"
}